{
  "gene_symbol": "HSPA4",
  "term_label": "protein folding",
  "gene_name": "Heat shock 70 kDa protein 4",
  "term_id": "GO:0006457",
  "gene": "UniProtKB:P34932"
}